{
  "gene_name": "Epimerase family protein SDR39U1",
  "term_id": "UNKNOWN:0003",
  "gene": "UniProtKB:Q9NRG7",
  "gene_symbol": "SDR39U1",
  "term_label": "Unknown cellular component"
}